rRNA modification [GO:0000154] (biological process) Definition: The covalent alteration of one or more nucleotides within an rRNA molecule to produce an rRNA molecule with a sequence that differs from that coded genetically. Sources: GOC:curators Note: The term 'RNA editing' (GO:0016547) was merged into 'RNA modification' (GO:0009451) on the basis of statements in the preface of Modification and Editing of RNA (ISBN:1555811337) that there is no clear distinction between modification and editing. Parallel changes were made for substrate (e.g. tRNA, rRNA, etc.) specific child terms of 'RNA editing'. Also known as: rRNA editing Subtypes: cotranscriptional mitochondrial rRNA nucleotide insertion [GO:0002110], rRNA pseudouridine synthesis [GO:0031118], rRNA methylation [GO:0031167], rRNA acetylation [GO:1990882] Relationships: is a type of rRNA processing [GO:0006364]; is a type of GO:0009451